positive regulation of cellotriose catabolic process [GO:2000938] (biological process) Relationships: is a type of GO:0009896; is a type of positive regulation of carbohydrate metabolic process [GO:0045913]; is a type of regulation of cellotriose catabolic process [GO:2000936]; positively regulates cellotriose catabolic process [GO:2000894] Definition: Any process that activates or increases the frequency, rate or extent of cellotriose catabolic process. Sources: GOC:mengo_curators Also known as: positive regulation of cellotriose catabolism